{
  "gene": "UniProtKB:Q9Y3E7",
  "gene_symbol": "CHMP3",
  "term_id": "GO:0005771",
  "term_label": "multivesicular body",
  "gene_name": "Charged multivesicular body protein 3"
}